{
  "term_id": "GO:0006487",
  "term_label": "protein N-linked glycosylation",
  "gene": "UniProtKB:Q92871",
  "gene_name": "Phosphomannomutase 1",
  "gene_symbol": "PMM1"
}